positive regulation of smooth endoplasmic reticulum calcium ion concentration [GO:0051564] (biological process) Definition: Any process that increases the concentration of calcium ions in the smooth endoplasmic reticulum. Relationships: is a type of positive regulation of endoplasmic reticulum calcium ion concentration [GO:0032470]; is a type of smooth endoplasmic reticulum calcium ion homeostasis [GO:0051563] Also known as: elevation of calcium ion concentration in smooth endoplasmic reticulum, elevation of smooth ER calcium ion concentration, elevation of smooth endoplasmic reticulum calcium ion concentration, smooth endoplasmic reticulum calcium ion concentration elevation Sources: GOC:ai